{
  "gene": "UniProtKB:Q5JSH3",
  "term_label": "regulation of vesicle-mediated transport",
  "gene_symbol": "WDR44",
  "gene_name": "WD repeat-containing protein 44",
  "term_id": "GO:0060627"
}